{
  "term_label": "Unknown cellular component",
  "gene_name": "Cyclic nucleotide-binding domain-containing protein 1",
  "term_id": "UNKNOWN:0003",
  "gene_symbol": "CNBD1",
  "gene": "UniProtKB:Q8NA66"
}